metanephric distal convoluted tubule development [GO:0072221] (biological process) Relationships: is a type of GO:0072025; is a type of GO:0072234; is part of metanephric distal tubule development [GO:0072235] Sources: GOC:mtg_kidney_jan10 Definition: The process whose specific outcome is the progression of the metanephric distal convoluted tubule over time, from its formation to the mature structure. The metanephric distal convoluted tubule is the first segment of the metanephric nephron lying just downstream from the loop of Henle, immediately after the macula densa. Among other functions, in humans it is responsible for the reabsorption of about 5% of filtered sodium via the thiazide-sensitive Na-Cl symporter.